{
  "gene_name": "Erythroid transcription factor",
  "term_label": "RNA polymerase II cis-regulatory region sequence-specific DNA binding",
  "gene": "UniProtKB:P15976",
  "gene_symbol": "GATA1",
  "term_id": "GO:0000978"
}